{
  "gene_name": "Secretory carrier-associated membrane protein 2",
  "term_id": "GO:0032588",
  "gene": "UniProtKB:O15127",
  "term_label": "trans-Golgi network membrane",
  "gene_symbol": "SCAMP2"
}